{
  "term_id": "GO:0045893",
  "gene_name": "Myelin regulatory factor",
  "term_label": "positive regulation of DNA-templated transcription",
  "gene_symbol": "MYRF",
  "gene": "UniProtKB:Q9Y2G1"
}